{
  "term_id": "GO:0000226",
  "term_label": "microtubule cytoskeleton organization",
  "gene": "UniProtKB:O75147",
  "gene_symbol": "OBSL1",
  "gene_name": "Obscurin-like protein 1"
}